{
  "gene_name": "TPT1-like protein",
  "gene_symbol": "Q56UQ5",
  "gene": "UniProtKB:Q56UQ5",
  "term_id": "GO:0005509",
  "term_label": "calcium ion binding"
}